ADP-specific phosphofructokinase activity [GO:0043844] (molecular function) Also known as: ADP-6-phosphofructokinase activity, ADP-Pfk activity, ADP-dependent phosphofructokinase activity, ADP:D-fructose-6-phosphate 1-phosphotransferase activity Relationships: is a type of kinase activity [GO:0016301]; is a type of GO:0016773 Sources: EC:2.7.1.146 Definition: Catalysis of the reaction: ADP + D-fructose 6-phosphate = AMP + D-fructose 1,6-bisphosphate.